{
  "gene_symbol": "LINC02876",
  "gene_name": "Uncharacterized protein encoded by LINC02876",
  "gene": "UniProtKB:F2Z3M2",
  "term_label": "Unknown cellular component",
  "term_id": "UNKNOWN:0003"
}